{
  "term_label": "ubiquitin protein ligase activity",
  "gene_name": "E3 ubiquitin-protein ligase RNF38",
  "gene_symbol": "RNF38",
  "term_id": "GO:0061630",
  "gene": "UniProtKB:Q9H0F5"
}